Bergmann glial cell differentiation [GO:0060020] (biological process) References: PMID:10375501 Sources: GOC:dph Relationships: is a type of GO:0048708 Definition: The process in which neuroepithelial cells of the neural tube give rise to Brgmann glial cells, specialized bipotential progenitors cells of the cerebellum. Differentiation includes the processes involved in commitment of a cell to a specific fate.